cellular response to bacterial lipoprotein [GO:0071220] (biological process) Relationships: is a type of response to bacterial lipoprotein [GO:0032493]; is a type of GO:0071219 Definition: Any process that results in a change in state or activity of a cell (in terms of movement, secretion, enzyme production, gene expression, etc.) as a result of a bacterial lipoprotein stimulus. Sources: GOC:mah Subtypes: GO:0071221